{
  "gene_symbol": "ADGRL3",
  "gene_name": "Adhesion G protein-coupled receptor L3",
  "term_id": "GO:0005911",
  "term_label": "cell-cell junction",
  "gene": "UniProtKB:Q9HAR2"
}